{
  "gene_name": "Cylicin-2",
  "term_label": "Unknown molecular function",
  "gene_symbol": "CYLC2",
  "gene": "UniProtKB:Q14093",
  "term_id": "UNKNOWN:0001"
}